response to beta-carotene [GO:1905387] (biological process) Also known as: response to beta,beta-carotene Subtypes: cellular response to beta-carotene [GO:1905388] References: PMID:16771696 Sources: GOC:TermGenie, GO_REF:0000071 Relationships: is a type of GO:0033993 Definition: Any process that results in a change in state or activity of a cell or an organism (in terms of movement, secretion, enzyme production, gene expression, etc.) as a result of a beta-carotene stimulus.